{
  "gene_name": "Putative uncharacterized protein ENSP00000381562",
  "gene": "UniProtKB:A8MU10",
  "term_label": "Unknown cellular component",
  "gene_symbol": "A8MU10",
  "term_id": "UNKNOWN:0003"
}